alpha,alpha-trehalase activity [GO:0004555] (molecular function) Relationships: is_a trehalase activity [GO:0015927] References: PMID:19897915 Sources: RHEA:32675 Definition: Catalysis of the reaction: alpha,alpha-trehalose + H2O = 2 D-glucose. Also known as: alpha,alpha-trehalose glucohydrolase activity